{
  "gene_name": "Transcription factor HES-4",
  "term_id": "GO:0009952",
  "gene": "UniProtKB:Q9HCC6",
  "term_label": "anterior/posterior pattern specification",
  "gene_symbol": "HES4"
}